{
  "term_label": "regulation of transcription by RNA polymerase II",
  "gene": "UniProtKB:Q8NHY6",
  "gene_symbol": "ZFP28",
  "gene_name": "Zinc finger protein 28 homolog",
  "term_id": "GO:0006357"
}